negative regulation of tolerance induction to tumor cell [GO:0002844] (biological process) Also known as: down regulation of tolerance induction to tumor cell, down-regulation of tolerance induction to tumor cell, downregulation of tolerance induction to tumor cell, negative regulation of tolerance induction to tumour cell, inhibition of tolerance induction to tumor cell Sources: GOC:add Subtypes: GO:0002847 Relationships: is a type of negative regulation of peripheral tolerance induction [GO:0002659]; is a type of GO:0002838; is a type of GO:0002843; negatively regulates tolerance induction to tumor cell [GO:0002413] Definition: Any process that stops, prevents, or reduces the frequency, rate, or extent of tolerance induction to tumor cell.